geranylgeranyl diphosphate catabolic process [GO:1902247] (biological process) Definition: The chemical reactions and pathways resulting in the breakdown of geranylgeranyl diphosphate. Relationships: is a type of GO:0009395; is a type of terpenoid catabolic process [GO:0016115]; is a type of geranylgeranyl diphosphate metabolic process [GO:0033385] References: PMID:22672125 Sources: GOC:TermGenie Also known as: geranylgeranyl diphosphate breakdown, geranylgeranyl diphosphate catabolism, geranylgeranyl diphosphate degradation